symbiont-mediated perturbation of host cell motility [GO:1903653] (BP) Definition: A process in which a symbiont alters or subverts cell motility in its host organism. The host is defined as the larger of the organisms involved in a symbiotic interaction. References: PMID:25049409 Sources: GOC:TermGenie, GO_REF:0000063 Also known as: modulation by symbiont of host cell locomotion, modulation by symbiont of host cell motility, regulation by symbiont of host cell motility, modulation by symbiont of host cell movement Relationships: is a type of symbiont-mediated perturbation of host cellular process [GO:0044068]